negative regulation of G2/MI transition of meiotic cell cycle [GO:0110031] (biological process) Definition: Any signaling pathway that decreases or inhibits the activity of a cell cycle cyclin-dependent protein kinase to modulate the switch from G2 phase to MI phase of the meiotic cell cycle. Subtypes: meiotic G2/MI DNA replication checkpoint signaling [GO:0033315] References: PMID:25492408 Sources: GOC:vw Relationships: is a type of GO:0110030; is a type of negative regulation of meiotic cell cycle phase transition [GO:1901994]; is a type of GO:1902750; negatively regulates G2/MI transition of meiotic cell cycle [GO:0008315]